regulation of hematopoietic stem cell migration [GO:2000471] (biological process) Also known as: regulation of hemopoietic stem cell migration Subtypes: negative regulation of hematopoietic stem cell migration [GO:2000472], positive regulation of hematopoietic stem cell migration [GO:2000473] Definition: Any process that modulates the frequency, rate or extent of hematopoietic stem cell migration. Sources: GOC:obol Relationships: is a type of regulation of cell migration [GO:0030334]; regulates GO:0035701